regulation of mitochondrial depolarization [GO:0051900] (BP) Relationships: is a type of regulation of membrane depolarization [GO:0003254]; is a type of regulation of mitochondrial membrane potential [GO:0051881]; regulates mitochondrial depolarization [GO:0051882] Definition: Any process that modulates the frequency, rate or extent of the change in the membrane potential of the mitochondria from negative to positive. Sources: GOC:ai Subtypes: positive regulation of mitochondrial depolarization [GO:0051901], GO:0051902